{
  "term_label": "olfactory receptor activity",
  "term_id": "GO:0004984",
  "gene_symbol": "OR52B6",
  "gene_name": "Olfactory receptor 52B6",
  "gene": "UniProtKB:Q8NGF0"
}